positive regulation of lipid localization [GO:1905954] (biological process) Definition: Any process that activates or increases the frequency, rate or extent of lipid localization. Relationships: is a type of positive regulation of biological process [GO:0048518]; is a type of regulation of lipid localization [GO:1905952]; positively regulates lipid localization [GO:0010876] Subtypes: positive regulation of lipid storage [GO:0010884], positive regulation of lipid transport [GO:0032370] Also known as: positive regulation of lipid localisation, up regulation of lipid localisation, up regulation of lipid localization, up-regulation of lipid localisation, up-regulation of lipid localization, upregulation of lipid localisation, upregulation of lipid localization, activation of lipid localisation, activation of lipid localization References: PMID:17564681 Sources: GOC:TermGenie, GO_REF:0000058